{
  "gene_symbol": "ARL8B",
  "term_id": "GO:0008089",
  "gene": "UniProtKB:Q9NVJ2",
  "gene_name": "ADP-ribosylation factor-like protein 8B",
  "term_label": "anterograde axonal transport"
}